{
  "gene": "UniProtKB:Q8NFI4",
  "term_id": "UNKNOWN:0003",
  "gene_name": "Putative protein FAM10A5",
  "term_label": "Unknown cellular component",
  "gene_symbol": "ST13P5"
}